{
  "gene": "UniProtKB:Q9BPZ2",
  "term_label": "regulation of DNA-templated transcription",
  "gene_symbol": "SPIN2B",
  "gene_name": "Spindlin-2B",
  "term_id": "GO:0006355"
}